{
  "term_label": "cytoplasm",
  "gene_symbol": "YTHDF1",
  "term_id": "GO:0005737",
  "gene_name": "YTH domain-containing family protein 1",
  "gene": "UniProtKB:Q9BYJ9"
}